arylalkyl acylamidase activity [GO:0047416] (molecular function) Also known as: N-acetylarylalkylamine amidohydrolase activity, aralkyl acylamidase activity Relationships: is a type of GO:0016811 Definition: Catalysis of the reaction: H2O + N-acetylarylalkylamine = acetate + arylalkylamine. Sources: EC:3.5.1.76, MetaCyc:3.5.1.76-RXN